{
  "term_label": "protein targeting to vacuole",
  "gene_name": "Vacuolar protein sorting-associated protein 37A",
  "gene_symbol": "VPS37A",
  "gene": "UniProtKB:Q8NEZ2",
  "term_id": "GO:0006623"
}